{
  "gene": "UniProtKB:Q9NXF1",
  "gene_symbol": "TEX10",
  "term_id": "GO:0005634",
  "gene_name": "Testis-expressed protein 10",
  "term_label": "nucleus"
}